{
  "gene_symbol": "CUZD1",
  "gene": "UniProtKB:Q86UP6",
  "gene_name": "CUB and zona pellucida-like domain-containing protein 1",
  "term_id": "UNKNOWN:0002",
  "term_label": "Unknown biological process"
}